{
  "term_label": "endoplasmic reticulum",
  "gene_name": "Mannosyl-oligosaccharide 1,2-alpha-mannosidase IB",
  "gene_symbol": "MAN1A2",
  "gene": "UniProtKB:O60476",
  "term_id": "GO:0005783"
}